{
  "gene_name": "Putative beta-lactamase-like 1",
  "gene": "UniProtKB:A8MY62",
  "gene_symbol": "LACTBL1",
  "term_id": "UNKNOWN:0001",
  "term_label": "Unknown molecular function"
}